{
  "gene_symbol": "CTNNBIP1",
  "term_label": "beta-catenin binding",
  "term_id": "GO:0008013",
  "gene": "UniProtKB:Q9NSA3",
  "gene_name": "Beta-catenin-interacting protein 1"
}